ovarian follicle development [GO:0001541] (biological process) Definition: The process whose specific outcome is the progression of the ovarian follicle over time, from its formation to the mature structure. Relationships: is a type of anatomical structure development [GO:0048856]; BFO_0000050 female gonad development [GO:0008585] Also known as: follicular phase Regulation: regulated by regulation of ovarian follicle development [GO:2000354]; negatively regulated by negative regulation of ovarian follicle development [GO:2000355]; positively regulated by GO:2000386 Sources: https://www.ncbi.nlm.nih.gov/books/NBK279054/